{
  "gene": "UniProtKB:Q58F21",
  "term_label": "nucleus",
  "gene_symbol": "BRDT",
  "term_id": "GO:0005634",
  "gene_name": "Bromodomain testis-specific protein"
}